norepinephrine uptake [GO:0051620] (biological process) Also known as: levarterenol reuptake, levarterenol uptake, noradrenaline reuptake, noradrenaline uptake, norepinephrine import, norepinephrine reuptake Relationships: is a type of GO:0015874; is a type of catecholamine uptake [GO:0090493] Regulation: regulated by regulation of norepinephrine uptake [GO:0051621]; negatively regulated by negative regulation of norepinephrine uptake [GO:0051622]; positively regulated by positive regulation of norepinephrine uptake [GO:0051623] Sources: GOC:ai Definition: The directed movement of norepinephrine into a cell, typically presynaptic neurons or glial cells. Norepinephrine (3,4-dihydroxyphenyl-2-aminoethanol) is a hormone secreted by the adrenal medulla and a neurotransmitter in the sympathetic peripheral nervous system and in some tracts of the CNS. It is also the biosynthetic precursor of epinephrine.